aryl hydrocarbon receptor complex [GO:0034751] (cellular component) Definition: A protein complex that acts as an aryl hydrocarbon (Ah) receptor. Cytosolic and nuclear Ah receptor complexes have different subunit composition, but both contain the ligand-binding subunit AhR. References: PMID:7598497 Sources: GOC:mah Subtypes: cytosolic aryl hydrocarbon receptor complex [GO:0034752], nuclear aryl hydrocarbon receptor complex [GO:0034753] Relationships: is a type of receptor complex [GO:0043235]; is a type of intracellular protein-containing complex [GO:0140535] Also known as: AHRC, AhR complex